interleukin4-interleukin-4 receptor complex [GO:0070450] (cellular component) Also known as: IL4-IL4 receptor complex, IL4-IL4R-IL2RG complex Definition: A protein complex that is formed by the association of a heterodimeric interleukin-4 receptor complex with an interleukin-4 molecule. References: PMID:10358772 Sources: GOC:mah Relationships: is a type of plasma membrane protein complex [GO:0098797]